{
  "gene_name": "Syntaxin-12",
  "term_id": "GO:0012505",
  "gene_symbol": "STX12",
  "gene": "UniProtKB:Q86Y82",
  "term_label": "endomembrane system"
}